{
  "term_label": "site of double-strand break",
  "gene": "UniProtKB:Q8N884",
  "gene_symbol": "CGAS",
  "term_id": "GO:0035861",
  "gene_name": "Cyclic GMP-AMP synthase"
}